{
  "gene": "UniProtKB:Q8TDC0",
  "term_id": "GO:0003779",
  "gene_name": "Myozenin-3",
  "term_label": "actin binding",
  "gene_symbol": "MYOZ3"
}